{
  "term_id": "GO:0051959",
  "gene_name": "Dynein axonemal heavy chain 17",
  "term_label": "dynein light intermediate chain binding",
  "gene_symbol": "DNAH17",
  "gene": "UniProtKB:Q9UFH2"
}